{
  "gene_symbol": "UTP14A",
  "term_id": "GO:0032040",
  "gene": "UniProtKB:Q9BVJ6",
  "term_label": "small-subunit processome",
  "gene_name": "U3 small nucleolar RNA-associated protein 14 homolog A"
}